homogentisate catabolic process [GO:1902000] (biological process) Definition: The chemical reactions and pathways resulting in the breakdown of homogentisate. References: PMID:22980205 Sources: GOC:TermGenie Relationships: is a type of phenol-containing compound catabolic process [GO:0019336]; is_a benzene-containing compound metabolic process [GO:0042537]; is a type of monocarboxylic acid catabolic process [GO:0072329] Also known as: homogentisate breakdown, homogentisate catabolism, homogentisate degradation